regulation of compound eye photoreceptor cell differentiation [GO:0110116] (biological process) Definition: Any process that modulates the frequency, rate or extent of compound eye photoreceptor cell differentiation. References: PMID:16377567 Sources: GOC:ha Relationships: is a type of regulation of photoreceptor cell differentiation [GO:0046532]; regulates compound eye photoreceptor cell differentiation [GO:0001751] Subtypes: regulation of R7 cell differentiation [GO:0045676], regulation of R8 cell differentiation [GO:0045679], positive regulation of compound eye photoreceptor cell differentiation [GO:0110117], negative regulation of compound eye photoreceptor cell differentiation [GO:0110118]